{
  "gene_symbol": "SCAI",
  "term_label": "nucleus",
  "gene": "UniProtKB:Q8N9R8",
  "term_id": "GO:0005634",
  "gene_name": "Protein SCAI"
}